negative regulation of inflammatory response to antigenic stimulus [GO:0002862] (biological process) Also known as: down regulation of inflammatory response to antigenic stimulus, down-regulation of inflammatory response to antigenic stimulus, downregulation of inflammatory response to antigenic stimulus, inhibition of inflammatory response to antigenic stimulus Definition: Any process that stops, prevents, or reduces the frequency, rate, or extent of an inflammatory response to an antigenic stimulus. Sources: GOC:add Subtypes: negative regulation of acute inflammatory response to antigenic stimulus [GO:0002865], negative regulation of chronic inflammatory response to antigenic stimulus [GO:0002875] Relationships: is a type of regulation of inflammatory response to antigenic stimulus [GO:0002861]; is_a negative regulation of inflammatory response [GO:0050728]; is a type of negative regulation of immune response [GO:0050777]; RO_0002212 inflammatory response to antigenic stimulus [GO:0002437]